response to cocaine [GO:0042220] (biological process) Subtypes: GO:0071314 Definition: Any process that results in a change in state or activity of a cell or an organism (in terms of movement, secretion, enzyme production, gene expression, etc.) as a result of a cocaine stimulus. Cocaine is a crystalline alkaloid obtained from the leaves of the coca plant. Sources: GOC:ef, GOC:jl Relationships: is a type of response to alkaloid [GO:0043279]; is a type of GO:1901700